negative regulation of cobalamin metabolic process [GO:0106122] (biological process) Relationships: is a type of negative regulation of metabolic process [GO:0009892]; is a type of regulation of cobalamin metabolic process [GO:0106064]; RO_0002212 cobalamin metabolic process [GO:0009235] Definition: Any process that stops, prevents or reduces the frequency, rate or extent of a cobalamin metabolic process. References: PMID:29056341